{
  "gene_symbol": "NCOA3",
  "term_label": "positive regulation of transcription by RNA polymerase II",
  "term_id": "GO:0045944",
  "gene_name": "Nuclear receptor coactivator 3",
  "gene": "UniProtKB:Q9Y6Q9"
}